{
  "gene_name": "Brain-specific angiogenesis inhibitor 1-associated protein 2-like protein 2",
  "term_label": "actin filament bundle assembly",
  "gene_symbol": "BAIAP2L2",
  "gene": "UniProtKB:Q6UXY1",
  "term_id": "GO:0051017"
}